{
  "gene": "UniProtKB:P22362",
  "gene_name": "C-C motif chemokine 1",
  "term_label": "antimicrobial humoral immune response mediated by antimicrobial peptide",
  "gene_symbol": "CCL1",
  "term_id": "GO:0061844"
}